{
  "term_id": "GO:0140326",
  "term_label": "ATPase-coupled intramembrane lipid transporter activity",
  "gene_symbol": "ATP9B",
  "gene_name": "Probable phospholipid-transporting ATPase IIB",
  "gene": "UniProtKB:O43861"
}